{
  "gene": "UniProtKB:Q8IWI9",
  "term_id": "GO:0006357",
  "gene_symbol": "MGA",
  "gene_name": "MAX gene-associated protein",
  "term_label": "regulation of transcription by RNA polymerase II"
}